{
  "gene_name": "RNA-binding region-containing protein 3",
  "term_id": "GO:0000398",
  "gene_symbol": "RNPC3",
  "gene": "UniProtKB:Q96LT9",
  "term_label": "mRNA splicing, via spliceosome"
}